{
  "gene": "UniProtKB:Q15761",
  "term_label": "pancreatic polypeptide receptor activity",
  "gene_name": "Neuropeptide Y receptor type 5",
  "term_id": "GO:0001602",
  "gene_symbol": "NPY5R"
}